{
  "term_id": "GO:0005666",
  "gene": "UniProtKB:O75575",
  "term_label": "RNA polymerase III complex",
  "gene_symbol": "CRCP",
  "gene_name": "DNA-directed RNA polymerase III subunit RPC9"
}